{
  "gene": "UniProtKB:Q9NS82",
  "gene_name": "Asc-type amino acid transporter 1",
  "term_label": "L-amino acid transmembrane transporter activity",
  "gene_symbol": "SLC7A10",
  "term_id": "GO:0015179"
}